lipoprotein lipid oxidation [GO:0034439] (biological process) Definition: The modification of a lipoprotein by oxidation of the lipid group. Sources: GOC:BHF, GOC:mah Relationships: is a type of GO:0034440; is a type of GO:0042161 Regulation: regulated by regulation of lipoprotein lipid oxidation [GO:0060587]; RO_0002212 by negative regulation of lipoprotein lipid oxidation [GO:0060588]